{
  "gene": "UniProtKB:A0PK00",
  "term_id": "UNKNOWN:0001",
  "term_label": "Unknown molecular function",
  "gene_symbol": "TMEM120B",
  "gene_name": "Transmembrane protein 120B"
}